{
  "gene": "UniProtKB:Q92522",
  "term_label": "double-stranded DNA binding",
  "gene_symbol": "H1-10",
  "term_id": "GO:0003690",
  "gene_name": "Histone H1.10"
}